{
  "term_label": "Unknown molecular function",
  "gene_name": "Acidic leucine-rich nuclear phosphoprotein 32 family member D",
  "term_id": "UNKNOWN:0001",
  "gene_symbol": "ANP32D",
  "gene": "UniProtKB:O95626"
}